trigeminal nerve morphogenesis [GO:0021636] (biological process) Also known as: CN V morphogenesis Sources: GOC:cls, GOC:dgh, GOC:dph, GOC:jid, GO_REF:0000021 Relationships: is a type of cranial nerve morphogenesis [GO:0021602]; is part of trigeminal nerve development [GO:0021559] Definition: The process in which the anatomical structure of the trigeminal nerve is generated and organized. The trigeminal nerve is composed of three large branches. They are the ophthalmic (V1, sensory), maxillary (V2, sensory) and mandibular (V3, motor and sensory) branches. The sensory ophthalmic branch travels through the superior orbital fissure and passes through the orbit to reach the skin of the forehead and top of the head. The maxillary nerve contains sensory branches that reach the pterygopalatine fossa via the inferior orbital fissure (face, cheek and upper teeth) and pterygopalatine canal (soft and hard palate, nasal cavity and pharynx). The motor part of the mandibular branch is distributed to the muscles of mastication, the mylohyoid muscle and the anterior belly of the digastric. The mandibular nerve also innervates the tensor veli palatini and tensor tympani muscles. The sensory part of the mandibular nerve is composed of branches that carry general sensory information from the mucous membranes of the mouth and cheek, anterior two-thirds of the tongue, lower teeth, skin of the lower jaw, side of the head and scalp and meninges of the anterior and middle cranial fossae.